{
  "gene_name": "MARVEL domain-containing protein 1",
  "term_label": "membrane",
  "term_id": "GO:0016020",
  "gene_symbol": "MARVELD1",
  "gene": "UniProtKB:Q9BSK0"
}